{
  "term_label": "sarcomere organization",
  "gene_symbol": "MYOM3",
  "term_id": "GO:0045214",
  "gene": "UniProtKB:Q5VTT5",
  "gene_name": "Myomesin-3"
}